{
  "term_id": "UNKNOWN:0002",
  "gene": "UniProtKB:Q9H0P7",
  "gene_name": "Putative uncharacterized protein encoded by AGPAT4-IT1",
  "gene_symbol": "AGPAT4-IT1",
  "term_label": "Unknown biological process"
}